protein localization to actin cytoskeleton [GO:1903119] (biological process) References: PMID:24798735 Sources: GOC:TermGenie, GO_REF:0000087 Subtypes: GO:0044379, GO:1903120, protein localization to actomyosin contractile ring [GO:1990179] Also known as: protein localisation in actin cytoskeleton, protein localisation to actin cytoskeleton, protein localization in actin cytoskeleton Definition: A process in which a protein is transported to, or maintained in, the location of an actin cytoskeleton. Relationships: is a type of protein localization to cytoskeleton [GO:0044380]